{
  "term_id": "GO:0005689",
  "gene_symbol": "SF3B2",
  "term_label": "U12-type spliceosomal complex",
  "gene_name": "Splicing factor 3B subunit 2",
  "gene": "UniProtKB:Q13435"
}